{
  "gene": "UniProtKB:Q9NRN7",
  "term_id": "GO:0008897",
  "term_label": "holo-[acyl-carrier-protein] synthase activity",
  "gene_symbol": "AASDHPPT",
  "gene_name": "L-aminoadipate-semialdehyde dehydrogenase-phosphopantetheinyl transferase"
}